{
  "term_id": "GO:0009897",
  "gene_symbol": "CLEC6A",
  "term_label": "external side of plasma membrane",
  "gene": "UniProtKB:Q6EIG7",
  "gene_name": "C-type lectin domain family 6 member A"
}